{
  "term_label": "RNA endonuclease activity",
  "term_id": "GO:0004521",
  "gene": "UniProtKB:Q9UKF6",
  "gene_name": "Cleavage and polyadenylation specificity factor subunit 3",
  "gene_symbol": "CPSF3"
}